{
  "gene_symbol": "PGAM5",
  "term_label": "positive regulation of mitochondrial fission",
  "gene": "UniProtKB:Q96HS1",
  "gene_name": "Serine_threonine-protein phosphatase PGAM5, mitochondrial",
  "term_id": "GO:0090141"
}